myosin II heavy chain binding [GO:0032038] (molecular function) Definition: Binding to a heavy chain of a myosin II complex. Relationships: is a type of myosin heavy chain binding [GO:0032036]; is a type of myosin II binding [GO:0045159] Sources: GOC:mah Subtypes: GO:0032034, myosin II tail binding [GO:0032035]